L-valine transmembrane transporter activity [GO:0005304] (molecular function) Also known as: L-valine transporter activity, isoleucine/valine:sodium symporter activity, leucine/isoleucine/valine porter activity, leucine/valine/isoleucine permease activity, valine/tyrosine/tryptophan permease activity Relationships: is a type of neutral L-amino acid transmembrane transporter activity [GO:0015175]; is a type of GO:0015179; is a type of branched-chain amino acid transmembrane transporter activity [GO:0015658]; is part of L-valine transmembrane transport [GO:1903785] Sources: GOC:ai, GOC:mtg_transport, ISBN:0815340729 Definition: Enables the transfer of L-valine from one side of a membrane to the other. L-valine is 2-amino-3-methylbutanoic acid.